pyrimidine nucleobase metabolic process [GO:0006206] (biological process) Relationships: is a type of GO:0009112; is a type of pyrimidine-containing compound metabolic process [GO:0072527] Also known as: pyrimidine base metabolic process, pyrimidine base metabolism, pyrimidine metabolic process, pyrimidine metabolism Definition: The chemical reactions and pathways involving pyrimidine nucleobases, 1,3-diazine, organic nitrogenous bases. Subtypes: pyrimidine nucleobase catabolic process [GO:0006208], GO:0019856, cytosine metabolic process [GO:0019858], thymine metabolic process [GO:0019859], uracil metabolic process [GO:0019860] Sources: GOC:go_curators Regulation: negatively regulated by negative regulation of pyrimidine nucleobase metabolic process [GO:0045984]; positively regulated by positive regulation of pyrimidine nucleobase metabolic process [GO:0045985]